locus ceruleus morphogenesis [GO:0021704] (biological process) Definition: The process in which the anatomical structure of the locus ceruleus is generated and organized. In mice, the locus ceruleus is a dense cluster of neurons within the dorsorostral pons. This nucleus is the major location of neurons that release norepinephrine throughout the brain, and is responsible for physiological responses to stress and panic. Sources: GOC:cls, GOC:dgh, GOC:dph, GOC:jid, GO_REF:0000021 Relationships: is a type of anatomical structure morphogenesis [GO:0009653]; is part of pons morphogenesis [GO:0021583]; BFO_0000050 locus ceruleus development [GO:0021703]